protein storage vacuole membrane [GO:0032586] (cellular component) Relationships: is a type of plant-type vacuole membrane [GO:0009705]; is part of protein storage vacuole [GO:0000326] Definition: The lipid bilayer surrounding a protein storage vacuole. Sources: GOC:mah